positive regulation of T cell antigen processing and presentation [GO:0002627] (biological process) Sources: GOC:add Also known as: positive regulation of T lymphocyte antigen processing and presentation, positive regulation of T-cell antigen processing and presentation, positive regulation of T-lymphocyte antigen processing and presentation, up regulation of T cell antigen processing and presentation, up-regulation of T cell antigen processing and presentation, upregulation of T cell antigen processing and presentation, activation of T cell antigen processing and presentation, stimulation of T cell antigen processing and presentation Definition: Any process that activates or increases the frequency, rate, or extent of T cell antigen processing and presentation. Relationships: is a type of positive regulation of antigen processing and presentation [GO:0002579]; is a type of GO:0002625; is a type of GO:0002711; positively regulates GO:0002457